{
  "gene_symbol": "CCDC117",
  "term_id": "UNKNOWN:0001",
  "term_label": "Unknown molecular function",
  "gene_name": "Coiled-coil domain-containing protein 117",
  "gene": "UniProtKB:Q8IWD4"
}